pyoverdine catabolic process [GO:0002050] (biological process) Definition: The chemical reactions and pathways resulting in the breakdown of the siderochrome pyoverdine. References: PMID:15317763 Relationships: is a type of amide metabolic process [GO:0043603]; is a type of siderophore catabolic process [GO:0046215]